{
  "term_label": "Unknown molecular function",
  "gene_name": "Transmembrane and ubiquitin-like domain-containing protein 2",
  "gene_symbol": "TMUB2",
  "term_id": "UNKNOWN:0001",
  "gene": "UniProtKB:Q71RG4"
}